negative regulation of T cell receptor signaling pathway [GO:0050860] (biological process) Sources: GOC:ai Relationships: is a type of regulation of T cell receptor signaling pathway [GO:0050856]; is a type of negative regulation of antigen receptor-mediated signaling pathway [GO:0050858]; negatively regulates GO:0050852 Subtypes: termination of T cell signal transduction [GO:0023022] Also known as: down regulation of T cell receptor signaling pathway, down-regulation of T cell receptor signaling pathway, downregulation of T cell receptor signaling pathway, negative regulation of T cell receptor signalling pathway, negative regulation of T lymphocyte receptor signaling pathway, negative regulation of T lymphocyte receptor signalling pathway, negative regulation of T-cell receptor signaling pathway, negative regulation of T-lymphocyte receptor signaling pathway, negative regulation of T-lymphocyte receptor signalling pathway, negative regulation of TCR signaling pathway, inhibition of T cell receptor signaling pathway Definition: Any process that stops, prevents, or reduces the frequency, rate or extent of signaling pathways initiated by the cross-linking of an antigen receptor on a T cell.